{
  "gene_symbol": "BLM",
  "gene": "UniProtKB:P54132",
  "term_id": "GO:0000723",
  "term_label": "telomere maintenance",
  "gene_name": "RecQ-like DNA helicase BLM"
}